{
  "term_label": "RNA stem-loop binding",
  "gene_name": "Endogenous retrovirus group K member 19 Pol protein",
  "term_id": "GO:0035613",
  "gene_symbol": "ERVK-19",
  "gene": "UniProtKB:Q9WJR5"
}